{
  "gene": "UniProtKB:Q13795",
  "gene_symbol": "ARFRP1",
  "gene_name": "ADP-ribosylation factor-related protein 1",
  "term_id": "GO:0005794",
  "term_label": "Golgi apparatus"
}